N-terminal peptidyl-glutamine acetylation [GO:0017192] (biological process) Sources: RESID:AA0045 Definition: The acetylation of a glutamine residue in protein to form the N5-methyl-L-glutamine derivative. The occurrence of this modification has not been confirmed. Its annotation in sequence databases is either due to the misidentification of 2-pyrrolidone-5-carboxylic acid, or to inappropriate homolog comparisons when proteolytic modification is more probable. Relationships: is a type of GO:0006474; is a type of peptidyl-glutamine modification [GO:0018199]